{
  "gene_symbol": "JAG2",
  "gene": "UniProtKB:Q9Y219",
  "term_id": "GO:0005112",
  "term_label": "Notch binding",
  "gene_name": "Protein jagged-2"
}